spongiome [GO:0062160] (cellular component) Definition: A cellular anatomical entity which is a network of tubules and vessicles and is part of the contractile vacuole complex. It is involved in the discharge of water externally. One of its functions is osmoregulatory. Relationships: is a type of GO:0110165; is part of GO:0062159 References: PMID:23890380